{
  "term_label": "2-oxoglutarate-dependent dioxygenase activity",
  "term_id": "GO:0016706",
  "gene_name": "2-oxoglutarate and iron-dependent oxygenase JMJD4",
  "gene_symbol": "JMJD4",
  "gene": "UniProtKB:Q9H9V9"
}